xenobiotic export from cell [GO:0046618] (BP) Definition: The directed movement of a xenobiotic from a cell, into the extracellular region. A xenobiotic is a compound foreign to the organism exposed to it. It may be synthesized by another organism (like ampicilin) or it can be a synthetic chemical. Subtypes: xenobiotic detoxification by transmembrane export across the plasma membrane [GO:1990961] Also known as: drug export, xenobiotic export Sources: GOC:go_curators, GOC:krc Relationships: is a type of xenobiotic transport [GO:0042908]; is a type of transmembrane transport [GO:0055085]; is a type of export from cell [GO:0140352]